{
  "term_id": "UNKNOWN:0003",
  "gene_name": "Leucine-rich single-pass membrane protein 1",
  "gene_symbol": "LSMEM1",
  "term_label": "Unknown cellular component",
  "gene": "UniProtKB:Q8N8F7"
}